{
  "gene": "UniProtKB:A0A1B0GUS4",
  "term_label": "ubiquitin-dependent protein catabolic process",
  "gene_name": "Ubiquitin-conjugating enzyme E2 L5",
  "gene_symbol": "UBE2L5",
  "term_id": "GO:0006511"
}